{
  "gene_name": "Histone H2B type 1-K",
  "term_label": "DNA binding",
  "gene": "UniProtKB:O60814",
  "gene_symbol": "H2BC12",
  "term_id": "GO:0003677"
}